{
  "term_label": "Unknown biological process",
  "gene_name": "Transmembrane protein 150C",
  "gene": "UniProtKB:B9EJG8",
  "gene_symbol": "TMEM150C",
  "term_id": "UNKNOWN:0002"
}